{
  "gene_name": "SEC23-interacting protein",
  "term_label": "Golgi apparatus",
  "term_id": "GO:0005794",
  "gene_symbol": "SEC23IP",
  "gene": "UniProtKB:Q9Y6Y8"
}